interleukin-6 binding [GO:0019981] (molecular function) Definition: Binding to interleukin-6. Sources: GOC:jl Relationships: is a type of growth factor binding [GO:0019838]; is a type of GO:0019955 Also known as: IL-6 binding